{
  "gene": "UniProtKB:Q86UF4",
  "gene_name": "Coiled-coil domain-containing protein 190",
  "term_label": "Unknown molecular function",
  "gene_symbol": "CCDC190",
  "term_id": "UNKNOWN:0001"
}